{
  "term_id": "GO:0005654",
  "gene_name": "Zinc finger and BTB domain-containing protein 32",
  "gene": "UniProtKB:Q9Y2Y4",
  "gene_symbol": "ZBTB32",
  "term_label": "nucleoplasm"
}